presynaptic dense core vesicle exocytosis [GO:0099525] (biological process) Definition: The secretion of molecules (e.g. neuropeptides and neuromodulators such as serotonin and dopamine) contained within a membrane-bounced dense in response to increased presynaptic cytosolic calcium levels. References: PMID:17553987, PMID:24653208 Relationships: is a type of calcium ion-regulated exocytosis of neurotransmitter [GO:0048791]; is a type of neuronal dense core vesicle exocytosis [GO:0099011] Subtypes: neuropeptide secretion from presynapse [GO:0099539] Regulation: regulated by GO:0099161